cellular response to food [GO:0071240] (biological process) Relationships: is a type of response to food [GO:0032094]; is a type of cellular response to chemical stimulus [GO:0070887] Definition: Any process that results in a change in state or activity of a cell (in terms of movement, secretion, enzyme production, gene expression, etc.) as a result of a food stimulus; food is anything which, when taken into the body, serves to nourish or build up the tissues or to supply body heat. Sources: GOC:mah